{
  "term_id": "GO:2001212",
  "gene_symbol": "ELMO3",
  "gene_name": "Engulfment and cell motility protein 3",
  "gene": "UniProtKB:Q96BJ8",
  "term_label": "regulation of vasculogenesis"
}